{
  "gene_symbol": "MLLT1",
  "term_id": "GO:0045893",
  "gene": "UniProtKB:Q03111",
  "term_label": "positive regulation of DNA-templated transcription",
  "gene_name": "Protein ENL"
}